{
  "gene": "UniProtKB:P03956",
  "term_id": "GO:0030198",
  "gene_name": "Interstitial collagenase",
  "gene_symbol": "MMP1",
  "term_label": "extracellular matrix organization"
}